{
  "gene": "UniProtKB:Q96PD6",
  "gene_name": "2-acylglycerol O-acyltransferase 1",
  "gene_symbol": "MOGAT1",
  "term_label": "diacylglycerol biosynthetic process",
  "term_id": "GO:0006651"
}